{
  "term_label": "Unknown biological process",
  "gene_symbol": "COG1",
  "term_id": "UNKNOWN:0002",
  "gene_name": "Conserved oligomeric Golgi complex subunit 1",
  "gene": "UniProtKB:Q8WTW3"
}